epithelial cell maturation involved in prostate gland development [GO:0060743] (biological process) Definition: The developmental process, independent of morphogenetic (shape) change, that is required for an epithelial cell of the prostate gland to attain its fully functional state. An epithelial cell is a cell usually found in a two-dimensional sheet with a free surface. Relationships: is a type of GO:0002070; is part of epithelial cell differentiation involved in prostate gland development [GO:0060742] Also known as: prostate gland epithelial cell development Sources: GOC:dph